{
  "term_id": "GO:0005829",
  "gene_symbol": "DNAJB5",
  "gene_name": "DnaJ homolog subfamily B member 5",
  "term_label": "cytosol",
  "gene": "UniProtKB:O75953"
}